chlorate transport [GO:0015702] (biological process) Definition: The directed movement of chlorate into, out of or within a cell, or between cells, by means of some agent such as a transporter or pore. Sources: GOC:krc Relationships: is a type of inorganic anion transport [GO:0015698]